detoxification of arsenic-containing substance [GO:0071722] (biological process) Definition: Any process that reduces or removes the toxicity of compounds containing arsenic, including arsenates, arsenites, and arsenides. These include transport of such compounds away from sensitive areas and to compartments or complexes whose purpose is sequestration of arsenic or arsenic-containing compounds. References: PMID:11313333, PMID:20221439 Sources: GOC:kmv Also known as: detoxification of arsenic Relationships: is a type of detoxification [GO:0098754]; is part of response to arsenic-containing substance [GO:0046685]